{
  "gene_name": "Phosphatidate cytidylyltransferase 1",
  "gene": "UniProtKB:Q92903",
  "term_label": "phosphatidate cytidylyltransferase activity",
  "term_id": "GO:0004605",
  "gene_symbol": "CDS1"
}